{
  "gene": "UniProtKB:Q16760",
  "gene_symbol": "DGKD",
  "term_label": "intracellular signal transduction",
  "gene_name": "Diacylglycerol kinase delta",
  "term_id": "GO:0035556"
}